core primosome complex [GO:1990098] (cellular component) References: PMID:21856207 Sources: GOC:bhm Definition: A protein-DNA complex containing at least one DNA helicase and one primase. Can also contain associated proteins. The helicase component continues to unwind the double-stranded DNA (dsDNA) and the primase component synthesizes a RNA primer during initiation or restart of replication. Note: The core primosome refers to a helicase-primase complex, and should not be confused with the more general GO term 'primosome complex ; GO:1990077'. Relationships: is a type of GO:1990077 Also known as: core primosome